tyrosine phenol-lyase activity [GO:0050371] (MF) Definition: Catalysis of the reaction: L-tyrosine + H2O = NH4 + phenol + pyruvate. Relationships: is a type of carbon-carbon lyase activity [GO:0016830] Also known as: L-tyrosine phenol-lyase (deaminating), L-tyrosine phenol-lyase (deaminating; pyruvate-forming), beta-tyrosinase activity Sources: EC:4.1.99.2, RHEA:21704